{
  "term_id": "GO:0002926",
  "term_label": "tRNA wobble base 5-methoxycarbonylmethyl-2-thiouridinylation",
  "gene_name": "Elongator complex protein 3",
  "gene_symbol": "ELP3",
  "gene": "UniProtKB:Q9H9T3"
}